{
  "term_label": "Unknown molecular function",
  "gene_symbol": "KANK2",
  "gene": "UniProtKB:Q63ZY3",
  "gene_name": "KN motif and ankyrin repeat domain-containing protein 2",
  "term_id": "UNKNOWN:0001"
}